{
  "gene": "UniProtKB:Q8N661",
  "gene_symbol": "TMEM86B",
  "gene_name": "Lysoplasmalogenase",
  "term_label": "membrane",
  "term_id": "GO:0016020"
}